{
  "gene": "UniProtKB:Q8NGR5",
  "term_id": "GO:0005886",
  "gene_symbol": "OR1L4",
  "term_label": "plasma membrane",
  "gene_name": "Olfactory receptor 1L4"
}